{
  "term_id": "GO:0003712",
  "gene": "UniProtKB:Q8WYB5",
  "gene_name": "Histone acetyltransferase KAT6B",
  "term_label": "transcription coregulator activity",
  "gene_symbol": "KAT6B"
}